{
  "gene": "UniProtKB:Q9P2D1",
  "gene_symbol": "CHD7",
  "term_id": "GO:0140658",
  "gene_name": "Chromodomain-helicase-DNA-binding protein 7",
  "term_label": "ATP-dependent chromatin remodeler activity"
}